response to methotrexate [GO:0031427] (biological process) Subtypes: cellular response to methotrexate [GO:0071414] Relationships: is a type of response to nitrogen compound [GO:1901698]; is a type of response to oxygen-containing compound [GO:1901700] Sources: GOC:ef, GOC:mah, ISBN:0198506732 Definition: Any process that results in a change in state or activity of a cell or an organism (in terms of movement, secretion, enzyme production, gene expression, etc.) as a result of a methotrexate stimulus. Methotrexate is 4-amino-10-methylformic acid, a folic acid analogue that is a potent competitive inhibitor of dihydrofolate reductase.